{
  "term_label": "actin filament binding",
  "term_id": "GO:0051015",
  "gene": "UniProtKB:P26232",
  "gene_symbol": "CTNNA2",
  "gene_name": "Catenin alpha-2"
}